positive regulation of lipid transport [GO:0032370] (biological process) Also known as: up regulation of lipid transport, up-regulation of lipid transport, upregulation of lipid transport, activation of lipid transport, stimulation of lipid transport Subtypes: positive regulation of sterol transport [GO:0032373], positive regulation of intracellular lipid transport [GO:0032379], GO:0045973, GO:1901508, GO:1903002, GO:2000193, GO:2000833, positive regulation of androstenedione secretion [GO:2000839], positive regulation of dehydroepiandrosterone secretion [GO:2000842], GO:2000845, GO:2001140 Relationships: is a type of GO:0032368; is a type of GO:0051050; is a type of positive regulation of lipid localization [GO:1905954]; RO_0002213 GO:0006869 Definition: Any process that activates or increases the frequency, rate or extent of the directed movement of lipids into, out of or within a cell, or between cells, by means of some agent such as a transporter or pore. Sources: GOC:mah